embryonic development via the syncytial blastoderm [GO:0001700] (biological process) Sources: GOC:go_curators, GOC:mtg_sensu Relationships: is a type of embryo development ending in birth or egg hatching [GO:0009792] Definition: The process whose specific outcome is the progression of the embryo over time, from zygote formation through syncytial blastoderm to the hatching of the first instar larva. An example of this process is found in Drosophila melanogaster.